{
  "gene": "UniProtKB:Q15007",
  "term_label": "nucleus",
  "gene_symbol": "WTAP",
  "gene_name": "Pre-mRNA-splicing regulator WTAP",
  "term_id": "GO:0005634"
}